{
  "term_id": "GO:0097322",
  "gene": "UniProtKB:O94992",
  "gene_name": "Protein HEXIM1",
  "term_label": "7SK snRNA binding",
  "gene_symbol": "HEXIM1"
}